{
  "gene": "UniProtKB:Q13595",
  "gene_name": "Transformer-2 protein homolog alpha",
  "gene_symbol": "TRA2A",
  "term_label": "mRNA splicing, via spliceosome",
  "term_id": "GO:0000398"
}